{
  "gene_name": "GATOR complex protein NPRL3",
  "gene_symbol": "NPRL3",
  "gene": "UniProtKB:Q12980",
  "term_id": "UNKNOWN:0001",
  "term_label": "Unknown molecular function"
}